{
  "gene_symbol": "STEEP1",
  "gene": "UniProtKB:Q9H5V9",
  "term_id": "UNKNOWN:0001",
  "gene_name": "STING ER exit protein",
  "term_label": "Unknown molecular function"
}